{
  "term_label": "detoxification of copper ion",
  "gene": "UniProtKB:P0DM35",
  "term_id": "GO:0010273",
  "gene_name": "Metallothionein 1H-like protein 1",
  "gene_symbol": "MT1HL1"
}